{
  "gene": "UniProtKB:A6NHQ2",
  "term_id": "GO:0008649",
  "term_label": "rRNA methyltransferase activity",
  "gene_symbol": "FBLL1",
  "gene_name": "rRNA_tRNA 2'-O-methyltransferase fibrillarin-like protein 1"
}